{
  "gene": "UniProtKB:Q6L8G4",
  "term_id": "UNKNOWN:0003",
  "gene_name": "Keratin-associated protein 5-11",
  "gene_symbol": "KRTAP5-11",
  "term_label": "Unknown cellular component"
}